{
  "term_id": "GO:0004300",
  "gene": "UniProtKB:Q86YB7",
  "term_label": "enoyl-CoA hydratase activity",
  "gene_name": "Enoyl-CoA hydratase domain-containing protein 2, mitochondrial",
  "gene_symbol": "ECHDC2"
}